{
  "term_label": "actin filament organization",
  "gene_symbol": "HIP1",
  "gene": "UniProtKB:O00291",
  "gene_name": "Huntingtin-interacting protein 1",
  "term_id": "GO:0007015"
}